lactase activity [GO:0000016] (MF) References: PMID:12023280 Definition: Catalysis of the reaction: lactose + H2O = D-glucose + D-galactose. Also known as: lactose galactohydrolase activity Relationships: is_a GO:0004553